lipopolysaccharide-1,6-galactosyltransferase activity [GO:0008921] (molecular function) Relationships: is a type of UDP-galactosyltransferase activity [GO:0035250] Also known as: LPS-1,6-galactosyltransferase activity Sources: GOC:ai Definition: Catalysis of the reaction: UDP-galactose + lipopolysaccharide = UDP + 1,6 alpha-D-galactosyl-lipopolysaccharide.